{
  "term_id": "GO:0006294",
  "term_label": "nucleotide-excision repair, preincision complex assembly",
  "gene_symbol": "GTF2H5",
  "gene": "UniProtKB:Q6ZYL4",
  "gene_name": "General transcription factor IIH subunit 5"
}